{
  "gene_name": "Elongation of very long chain fatty acids protein 4",
  "term_id": "GO:0030148",
  "term_label": "sphingolipid biosynthetic process",
  "gene": "UniProtKB:Q9GZR5",
  "gene_symbol": "ELOVL4"
}